{
  "term_label": "intracellular signal transduction",
  "term_id": "GO:0035556",
  "gene": "UniProtKB:P52824",
  "gene_symbol": "DGKQ",
  "gene_name": "Diacylglycerol kinase theta"
}